symbiont-mediated suppression of host protein localization to phagocytic vesicle [GO:0036522] (biological process) References: PMID:25063865 Sources: GOC:PARL, GOC:bf Relationships: is a type of symbiont-mediated perturbation of host process [GO:0044003] Definition: A process in which a symbiont inhibits or disrupts the normal localization of a protein to the host phagosome. The host is defined as the larger of the organisms involved in a symbiotic interaction. Also known as: disruption of host protein localisation to phagosome, inhibition of host protein localisation to phagosome, negative regulation by symbiont of host protein localization to phagocytic vesicle, suppression of host protein localisation to phagosome